interleukin-25 receptor activity [GO:0045507] (molecular function) Relationships: is a type of interleukin-17 receptor activity [GO:0030368]; has part interleukin-25 binding [GO:0045511] Sources: GOC:jl, GOC:signaling Also known as: IL-25 receptor activity, IL-25R Definition: Combining with interleukin-25 and transmitting the signal from one side of the membrane to the other to initiate a change in cell activity.